{
  "gene": "UniProtKB:Q8N9B5",
  "term_label": "Arp2/3 complex binding",
  "gene_name": "Junction-mediating and -regulatory protein",
  "gene_symbol": "JMY",
  "term_id": "GO:0071933"
}